multimerin complex [GO:1990972] (cellular component) Also known as: EMILIN-3 complex, EMILIN-4 complex, Elastic microfibrillar interface 3 complex, Elastic microfibrillar interface 4 complex, Multimerin-1 complex, Multimerin-2 complex, Platelet glycoprotein Ia* complex, p155 complex Relationships: is a type of GO:0098637; is part of extracellular matrix [GO:0031012] Definition: Glycoprotein complex of the C1q/TNF superfamily involved in cell adhesion. A homotrimer that will combine to form supramolecular Multimerin structures. References: PMID:9454761 Sources: GOC:bhm Note: An example of this is Multimerin-1 in human (Q13201) in PMID:9454761.